{
  "gene_name": "Sphingosine 1-phosphate receptor 5",
  "gene": "UniProtKB:Q9H228",
  "term_label": "adenylate cyclase-activating G protein-coupled receptor signaling pathway",
  "gene_symbol": "S1PR5",
  "term_id": "GO:0007189"
}